UUC codon-amino acid adaptor activity [GO:0033402] (molecular function) Also known as: TTC codon-amino acid adaptor activity, phenylalanine tRNA Definition: A triplet codon-amino acid adaptor activity that recognizes a UUC codon. Note: Note that in the standard genetic code, TTC codes for phenylalanine. Sources: GOC:mah Relationships: is a type of triplet codon-amino acid adaptor activity [GO:0030533]